{
  "term_label": "positive regulation of TORC1 signaling",
  "gene": "UniProtKB:P11309",
  "gene_symbol": "PIM1",
  "term_id": "GO:1904263",
  "gene_name": "Serine_threonine-protein kinase pim-1"
}